atrioventricular canal morphogenesis [GO:1905222] (biological process) Also known as: AV canal morphogenesis, AVC morphogenesis, atrial canal morphogenesis, atrio-ventricular canal morphogenesis, canalis atrioventricularis morphogenesis, ependymal canal morphogenesis Relationships: is a type of anatomical structure morphogenesis [GO:0009653]; is part of GO:0036302 References: PMID:19703439 Sources: GOC:BHF, GOC:TermGenie, GOC:rl, GO_REF:0000083 Definition: The developmental process by which an atrioventricular canal is generated and organized.